{
  "gene_name": "ATP-dependent DNA_RNA helicase DHX36",
  "term_label": "cytoplasm",
  "term_id": "GO:0005737",
  "gene_symbol": "DHX36",
  "gene": "UniProtKB:Q9H2U1"
}